butane monooxygenase activity [GO:0036174] (molecular function) References: PMID:17526838, PMID:19383682 Sources: GOC:dh Definition: Catalysis of the reaction: butane + O2 + NAD(P)H + H+ = butanol + NAD(P)+ + H2O. Also known as: sBMO, soluble butane monooxygenase Relationships: is a type of oxidoreductase activity, acting on paired donors, with incorporation or reduction of molecular oxygen, reduced iron-sulfur protein as one donor, and incorporation of one atom of oxygen [GO:0016713]